muscle cell fate commitment [GO:0042693] (biological process) Sources: CL:0000187, GOC:go_curators Definition: The process in which the cellular identity of muscle cells is acquired and determined. Relationships: is a type of cell fate commitment [GO:0045165]; BFO_0000050 muscle cell differentiation [GO:0042692] Subtypes: cardiac muscle cell fate commitment [GO:0060923], vascular associated smooth muscle cell fate commitment [GO:0097081]